{
  "term_label": "Unknown cellular component",
  "gene_symbol": "SPR",
  "gene": "UniProtKB:P35270",
  "gene_name": "Sepiapterin reductase",
  "term_id": "UNKNOWN:0003"
}